{
  "gene_symbol": "PLEKHA5",
  "gene": "UniProtKB:Q9HAU0",
  "term_id": "GO:0005829",
  "gene_name": "Pleckstrin homology domain-containing family A member 5",
  "term_label": "cytosol"
}